male genitalia morphogenesis [GO:0048808] (biological process) Also known as: male genital morphogenesis Subtypes: imaginal disc-derived male genitalia morphogenesis [GO:0048803], nematode male tail mating organ morphogenesis [GO:0090597] Sources: GOC:ems, ISBN:0140512888 Definition: The process in which the anatomical structures of male genitalia are generated and organized. Relationships: is a type of GO:0035112; is a type of male anatomical structure morphogenesis [GO:0090598]; is part of male genitalia development [GO:0030539]